transaldolase activity [GO:0004801] (MF) Relationships: is a type of transketolase or transaldolase activity [GO:0016744] Definition: Catalysis of the reaction: sedoheptulose 7-phosphate + D-glyceraldehyde 3-phosphate = D-erythrose 4-phosphate + D-fructose 6-phosphate. Also known as: dihydroxyacetone transferase activity, dihydroxyacetonetransferase activity, glycerone transferase activity, sedoheptulose-7-phosphate:D-glyceraldehyde-3-phosphate glyceronetransferase activity References: PMID:7592346 Sources: RHEA:17053